regulation of toll-like receptor 5 signaling pathway [GO:0034147] (BP) Definition: Any process that modulates the frequency, rate, or extent of toll-like receptor 5 signaling pathway. References: PMID:16551253, PMID:17328678 Sources: GOC:add Also known as: regulation of TLR5 signaling pathway, regulation of toll-like receptor 5 signalling pathway Relationships: is a type of regulation of pattern recognition receptor signaling pathway [GO:0062207]; regulates GO:0034146 Subtypes: negative regulation of toll-like receptor 5 signaling pathway [GO:0034148], GO:0034149